{
  "gene": "UniProtKB:P26599",
  "term_label": "mRNA binding",
  "gene_symbol": "PTBP1",
  "gene_name": "Polypyrimidine tract-binding protein 1",
  "term_id": "GO:0003729"
}